{
  "gene_symbol": "ATP5ME",
  "gene": "UniProtKB:P56385",
  "term_id": "GO:0005739",
  "term_label": "mitochondrion",
  "gene_name": "ATP synthase subunit e, mitochondrial"
}